tumor necrosis factor (ligand) superfamily member 11 production [GO:0072535] (biological process) Regulation: regulated by regulation of tumor necrosis factor (ligand) superfamily member 11 production [GO:2000307]; RO_0002212 by negative regulation of tumor necrosis factor (ligand) superfamily member 11 production [GO:2000308]; positively regulated by GO:2000309 Also known as: RANKL production, TNFSF11 production, tumor necrosis factor ligand superfamily member 11 production Definition: The appearance of tumor necrosis factor superfamily member 11 (TNFSF11; RANKL) due to biosynthesis or secretion following a cellular stimulus, resulting in an increase in its intracellular or extracellular levels. Note: Note that this term is in the subset of terms that should not be used for direct gene product annotation. Instead, select one of the 'regulation' children terms. Sources: GOC:BHF, GOC:mah Relationships: is a type of tumor necrosis factor superfamily cytokine production [GO:0071706]